mitochondrial derivative [GO:0016007] (cellular component) Sources: GOC:ma Subtypes: GO:0016006, GO:0016008, minor mitochondrial derivative [GO:0016009] Definition: The major and minor mitochondrial derivatives are the mitochondria of the sperm tail and derive by the unfolding of the Nebenkern during flagellum elongation. Relationships: is a type of intracellular membrane-bounded organelle [GO:0043231]